{
  "gene_name": "Carboxypeptidase B2",
  "gene": "UniProtKB:Q96IY4",
  "term_id": "GO:0042730",
  "term_label": "fibrinolysis",
  "gene_symbol": "CPB2"
}